amygdala development [GO:0021764] (BP) Sources: GOC:cls, GOC:dgh, GOC:dph, GOC:jid, GO_REF:0000021 Relationships: is a type of anatomical structure development [GO:0048856]; is part of limbic system development [GO:0021761] Definition: The progression of the amygdala over time from its initial formation until its mature state. The amygdala is an almond-shaped set of neurons in the medial temporal lobe of the brain that play a key role in processing emotions such as fear and pleasure.